positive regulation of imaginal disc growth [GO:0045572] (biological process) Definition: Any process that activates or increases the frequency, rate or extent of imaginal disc growth. Sources: GOC:go_curators Also known as: up regulation of imaginal disc growth, up-regulation of imaginal disc growth, upregulation of imaginal disc growth, activation of imaginal disc growth, stimulation of imaginal disc growth Relationships: is a type of regulation of imaginal disc growth [GO:0045570]; is a type of positive regulation of developmental growth [GO:0048639]; positively regulates imaginal disc growth [GO:0007446]